jasmonic acid biosynthetic process [GO:0009695] (biological process) Regulation: regulated by regulation of jasmonic acid biosynthetic process [GO:0080141] References: PMID:33821356 Also known as: jasmonic acid anabolism, jasmonic acid biosynthesis, jasmonic acid formation, jasmonic acid synthesis Relationships: is a type of jasmonic acid metabolic process [GO:0009694]; is a type of long-chain fatty acid biosynthetic process [GO:0042759] Definition: The chemical reactions and pathways resulting in the formation of jasmonic acid, a fatty acid derivative.